{
  "gene": "UniProtKB:Q6RFH8",
  "term_id": "GO:0005634",
  "term_label": "nucleus",
  "gene_name": "Double homeobox protein 4C",
  "gene_symbol": "DUX4L9"
}